{
  "gene": "UniProtKB:Q8WUD4",
  "term_label": "Unknown biological process",
  "gene_symbol": "CCDC12",
  "gene_name": "Coiled-coil domain-containing protein 12",
  "term_id": "UNKNOWN:0002"
}